{
  "gene": "UniProtKB:Q9UKT4",
  "gene_symbol": "FBXO5",
  "gene_name": "F-box only protein 5",
  "term_id": "UNKNOWN:0001",
  "term_label": "Unknown molecular function"
}